type-I cohesin domain binding [GO:1990311] (molecular function) Relationships: is a type of protein domain specific binding [GO:0019904] Definition: Binding to a type-I cohesin domain of a protein. Type-I cohesin domain is the binding partner of type-I dockerin domain. References: PMID:23195689, PMID:24080387 Sources: GOC:mengo_curators